negative regulation of tetrapyrrole biosynthetic process from glutamate [GO:1901411] (biological process) Also known as: down regulation of tetrapyrrole anabolism from glutamate, down regulation of tetrapyrrole biosynthesis from glutamate, down regulation of tetrapyrrole biosynthetic process from glutamate, down regulation of tetrapyrrole formation from glutamate, down regulation of tetrapyrrole synthesis from glutamate, down-regulation of tetrapyrrole anabolism from glutamate, down-regulation of tetrapyrrole biosynthesis from glutamate, down-regulation of tetrapyrrole biosynthetic process from glutamate, down-regulation of tetrapyrrole formation from glutamate, down-regulation of tetrapyrrole synthesis from glutamate, downregulation of tetrapyrrole anabolism from glutamate, downregulation of tetrapyrrole biosynthesis from glutamate, downregulation of tetrapyrrole biosynthetic process from glutamate, downregulation of tetrapyrrole formation from glutamate, downregulation of tetrapyrrole synthesis from glutamate, inhibition of tetrapyrrole anabolism from glutamate, inhibition of tetrapyrrole biosynthesis from glutamate, inhibition of tetrapyrrole formation from glutamate, inhibition of tetrapyrrole synthesis from glutamate, negative regulation of tetrapyrrole anabolism from glutamate, negative regulation of tetrapyrrole biosynthesis from glutamate, negative regulation of tetrapyrrole formation from glutamate, negative regulation of tetrapyrrole synthesis from glutamate, inhibition of tetrapyrrole biosynthetic process from glutamate Relationships: is a type of regulation of tetrapyrrole biosynthetic process from glutamate [GO:1901410]; is a type of GO:1901464; is a type of negative regulation of glutamate metabolic process [GO:2000212]; negatively regulates tetrapyrrole biosynthetic process from glutamate [GO:0033526] Sources: GOC:TermGenie, GOC:mengo_curators Definition: Any process that stops, prevents or reduces the frequency, rate or extent of tetrapyrrole biosynthetic process from glutamate.